sensory perception of pain [GO:0019233] (biological process) Sources: GOC:curators Definition: The series of events required for an organism to receive a painful stimulus, convert it to a molecular signal, and recognize and characterize the signal. A painful stimulus is any physical or chemical event that has the potential to cause tissue damage (actual or perceived) and activates the nociceptive system. Subtypes: GO:0019234, sensory perception of slow pain [GO:0019235] Relationships: is a type of GO:0007600 Regulation: regulated by regulation of sensory perception of pain [GO:0051930]; RO_0002212 by negative regulation of sensory perception of pain [GO:1904057]; positively regulated by positive regulation of sensory perception of pain [GO:1904058] Also known as: perception of physiological pain, nociception